{
  "term_id": "GO:0005634",
  "gene_symbol": "SAMD1",
  "gene": "UniProtKB:Q6SPF0",
  "gene_name": "Sterile alpha motif domain-containing protein 1",
  "term_label": "nucleus"
}